{
  "gene_name": "Melanocortin receptor 5",
  "gene": "UniProtKB:P33032",
  "term_id": "GO:0005737",
  "gene_symbol": "MC5R",
  "term_label": "cytoplasm"
}